{
  "term_label": "sperm principal piece",
  "gene": "UniProtKB:Q8N0Y7",
  "term_id": "GO:0097228",
  "gene_name": "Probable phosphoglycerate mutase 4",
  "gene_symbol": "PGAM4"
}